cellular response to amphetamine [GO:0071419] (biological process) Relationships: is a type of response to amphetamine [GO:0001975]; is_a cellular response to amine stimulus [GO:0071418] Definition: Any process that results in a change in state or activity of a cell (in terms of movement, secretion, enzyme production, gene expression, etc.) as a result of an amphetamine stimulus. Amphetamines consist of a group of compounds related to alpha-methylphenethylamine. Sources: GOC:mah